{
  "gene_symbol": "RNF103",
  "gene": "UniProtKB:O00237",
  "term_label": "ubiquitin-protein transferase activity",
  "term_id": "GO:0004842",
  "gene_name": "E3 ubiquitin-protein ligase RNF103"
}